{
  "gene_symbol": "PRRG4",
  "term_label": "plasma membrane",
  "gene_name": "Transmembrane gamma-carboxyglutamic acid protein 4",
  "term_id": "GO:0005886",
  "gene": "UniProtKB:Q9BZD6"
}